[methyl-Co(III) methylamine-specific corrinoid protein]:coenzyme M methyltransferase activity [GO:0043833] (molecular function) Sources: RHEA:18773 Also known as: MT2-A, methylcobamide:CoM methyltransferase activity, methylcobamide:coenzyme M methyltransferase activity, methylamine-specific methylcobalamin:CoM methyltransferase activity, methylamine-specific methylcobalamin:coenzyme M methyltransferase activity, monomethylamine-specific methylcobalamin:coenzyme M methyltransferase activity Definition: Catalysis of the reaction: [methyl-Co(III) methylamine-specific corrinoid protein] + coenzyme M = [Co(I) methylamine-specific corrinoid protein] + H+ + methyl-coenzyme M. This reaction is the transfer of the methyl group from the methylated corrinoid cofactor of a methylamine corrinoid protein to coenzyme M. Relationships: is a type of GO:0008168 Note: This function is the second step in the pathway of methanogenesis from monomethylamine, dimethylamine and trimethylamine.